{
  "gene_name": "Nuclear distribution protein nudE-like 1",
  "gene": "UniProtKB:Q9GZM8",
  "term_id": "GO:0007020",
  "term_label": "microtubule nucleation",
  "gene_symbol": "NDEL1"
}